{
  "gene_name": "Embryonic polyadenylate-binding protein 2",
  "term_label": "poly(A) binding",
  "term_id": "GO:0008143",
  "gene": "UniProtKB:A6NDY0",
  "gene_symbol": "PABPN1L"
}